{
  "term_label": "external side of plasma membrane",
  "gene_symbol": "CD1B",
  "term_id": "GO:0009897",
  "gene": "UniProtKB:P29016",
  "gene_name": "T-cell surface glycoprotein CD1b"
}